{
  "term_id": "GO:0006508",
  "gene_symbol": "PGA4",
  "term_label": "proteolysis",
  "gene": "UniProtKB:P0DJD7",
  "gene_name": "Pepsin A-4"
}